{
  "term_label": "actin binding",
  "gene_symbol": "MYOZ1",
  "gene": "UniProtKB:Q9NP98",
  "term_id": "GO:0003779",
  "gene_name": "Myozenin-1"
}